response to interferon-alpha [GO:0035455] (biological process) References: PMID:11356686 Sources: GOC:sl Definition: Any process that results in a change in state or activity of a cell or an organism (in terms of movement, secretion, enzyme production, gene expression, etc.) as a result of an interferon-alpha stimulus. Interferon-alpha is a type I interferon. Subtypes: cellular response to interferon-alpha [GO:0035457] Relationships: is a type of GO:0034097 Also known as: response to leukocyte interferon, response to lymphoblast interferon, response to lymphoblastoid interferon, response to interferon alfa-n1, response to interferon alfa-n3